{
  "gene_name": "WD repeat-containing protein 38",
  "gene_symbol": "WDR38",
  "term_label": "Unknown biological process",
  "gene": "UniProtKB:Q5JTN6",
  "term_id": "UNKNOWN:0002"
}